{
  "gene_name": "Phosphoinositide 3-kinase adapter protein 1",
  "gene": "UniProtKB:Q6ZUJ8",
  "term_label": "phosphatidylinositol 3-kinase regulatory subunit binding",
  "term_id": "GO:0036312",
  "gene_symbol": "PIK3AP1"
}